{
  "term_id": "GO:0005737",
  "term_label": "cytoplasm",
  "gene_symbol": "TGM6",
  "gene_name": "Protein-glutamine gamma-glutamyltransferase 6",
  "gene": "UniProtKB:O95932"
}